{
  "term_id": "GO:0003712",
  "gene": "UniProtKB:Q6ZN01",
  "gene_name": "MEF2-activating motif and SAP domain-containing transcriptional regulator",
  "term_label": "transcription coregulator activity",
  "gene_symbol": "MAMSTR"
}